{
  "gene": "UniProtKB:Q9Y3X0",
  "gene_name": "Coiled-coil domain-containing protein 9",
  "gene_symbol": "CCDC9",
  "term_label": "Unknown cellular component",
  "term_id": "UNKNOWN:0003"
}